{
  "gene_name": "Coronin-2B",
  "gene_symbol": "CORO2B",
  "term_label": "focal adhesion assembly",
  "gene": "UniProtKB:Q9UQ03",
  "term_id": "GO:0048041"
}